dorsal vessel heart proper cell fate commitment [GO:0035053] (biological process) Relationships: is a type of cell fate commitment involved in pattern specification [GO:0060581]; is_a cardiac cell fate commitment [GO:0060911]; is part of GO:0035054 References: PMID:12397110 Sources: GOC:bf, GOC:mtg_sensu Definition: The commitment of dorsal vessel cardioblast cells to a heart proper cell fate and their capacity to differentiate into heart cells. An example of this process is found in Drosophila melanogaster.